{
  "gene": "UniProtKB:Q6ZUB0",
  "term_label": "Unknown cellular component",
  "gene_symbol": "SPATA31D4",
  "gene_name": "Spermatogenesis-associated protein 31D4",
  "term_id": "UNKNOWN:0003"
}